{
  "term_id": "GO:0005743",
  "gene": "UniProtKB:Q96I51",
  "gene_symbol": "RCC1L",
  "gene_name": "RCC1-like G exchanging factor-like protein",
  "term_label": "mitochondrial inner membrane"
}